{
  "gene_name": "Orofacial cleft 1 candidate gene 1 protein",
  "term_label": "Unknown molecular function",
  "term_id": "UNKNOWN:0001",
  "gene": "UniProtKB:Q8IZS5",
  "gene_symbol": "OFCC1"
}